{
  "gene_name": "Guanylate-binding protein 5",
  "term_label": "GTP binding",
  "term_id": "GO:0005525",
  "gene_symbol": "GBP5",
  "gene": "UniProtKB:Q96PP8"
}